erythromycin catabolic process [GO:1901114] (biological process) Sources: GOC:TermGenie, GOC:yaf, UniPathway:UPA00240 Relationships: is a type of GO:0030640; is a type of macrolide metabolic process [GO:0033067]; is a type of lactone catabolic process [GO:1901335] Also known as: erythromycin breakdown, erythromycin catabolism, erythromycin degradation Definition: The chemical reactions and pathways resulting in the breakdown of erythromycin.